regulation of muscle system process [GO:0090257] (biological process) Relationships: is a type of GO:0044057; regulates muscle system process [GO:0003012] Sources: GOC:dph, GOC:tb Definition: Any process that modulates the frequency, rate or extent of a muscle system process, a multicellular organismal process carried out by any of the organs or tissues in a muscle system. Subtypes: GO:0006937, regulation of muscle hypertrophy [GO:0014743], GO:0043502, regulation of relaxation of muscle [GO:1901077]